{
  "gene_symbol": "KY",
  "term_label": "cytoplasm",
  "gene_name": "Kyphoscoliosis peptidase",
  "gene": "UniProtKB:Q8NBH2",
  "term_id": "GO:0005737"
}